DNA (cytosine-5-)-methyltransferase activity, acting on CpG substrates [GO:0051718] (molecular function) Definition: Catalysis of the reaction: S-adenosyl-L-methionine + CpG (in DNA) = S-adenosyl-L-homocysteine + 5-MeCpG (in DNA). References: PMID:15689527 Relationships: is a type of DNA (cytosine-5-)-methyltransferase activity [GO:0003886] Also known as: HpaII methylase, HpaII' methylase, M.BsuRIa, M.BsuRIb